{
  "term_id": "GO:0005829",
  "gene_symbol": "CNDP1",
  "gene": "UniProtKB:Q96KN2",
  "gene_name": "Beta-Ala-His dipeptidase",
  "term_label": "cytosol"
}